{
  "gene_name": "MAP kinase-activated protein kinase 3",
  "term_label": "nucleus",
  "gene": "UniProtKB:Q16644",
  "gene_symbol": "MAPKAPK3",
  "term_id": "GO:0005634"
}